5'-3' exonuclease activity [GO:0008409] (molecular function) Definition: Catalysis of the hydrolysis of ester linkages within nucleic acids by removing nucleotide residues from the 5' end. Sources: GOC:ai Relationships: is a type of exonuclease activity [GO:0004527] Subtypes: 5'-3' RNA exonuclease activity [GO:0004534], 5'-3' DNA exonuclease activity [GO:0035312]